{
  "term_label": "Unknown biological process",
  "gene_name": "Pleiotrophin",
  "gene_symbol": "PTN",
  "term_id": "UNKNOWN:0002",
  "gene": "UniProtKB:P21246"
}